{
  "gene": "UniProtKB:P19021",
  "gene_name": "Peptidyl-glycine alpha-amidating monooxygenase",
  "term_label": "peptidylglycine monooxygenase activity",
  "term_id": "GO:0004504",
  "gene_symbol": "PAM"
}